eye photoreceptor cell fate commitment [GO:0042706] (biological process) Sources: GOC:mtg_sensu Relationships: is a type of photoreceptor cell fate commitment [GO:0046552]; is part of eye photoreceptor cell differentiation [GO:0001754] Definition: The process in which the developmental fate of a cell becomes restricted such that it will develop into an eye photoreceptor cell. A photoreceptor cell is a cell that responds to incident electromagnetic radiation. Different classes of photoreceptor have different spectral sensitivities and express different photosensitive pigments. Subtypes: compound eye photoreceptor fate commitment [GO:0001752], GO:0060220